{
  "gene": "UniProtKB:Q9UBY8",
  "gene_name": "Protein CLN8",
  "term_id": "GO:0007399",
  "term_label": "nervous system development",
  "gene_symbol": "CLN8"
}